{
  "term_id": "GO:0005737",
  "gene_name": "CCHC-type zinc finger nucleic acid binding protein",
  "term_label": "cytoplasm",
  "gene_symbol": "CNBP",
  "gene": "UniProtKB:P62633"
}